{
  "gene": "UniProtKB:A6NER0",
  "gene_symbol": "TBC1D3F",
  "term_label": "Unknown biological process",
  "term_id": "UNKNOWN:0002",
  "gene_name": "TBC1 domain family member 3F"
}